{
  "term_id": "GO:0140374",
  "term_label": "antiviral innate immune response",
  "gene_symbol": "ZDHHC11B",
  "gene": "UniProtKB:P0C7U3",
  "gene_name": "Probable palmitoyltransferase ZDHHC11B"
}